{
  "gene_name": "Apolipoprotein B-100",
  "term_id": "GO:0034361",
  "gene": "UniProtKB:P04114",
  "term_label": "very-low-density lipoprotein particle",
  "gene_symbol": "APOB"
}